regulation of tube lumen cavitation [GO:1903132] (biological process) Relationships: is a type of regulation of developmental process [GO:0050793]; regulates tube lumen cavitation [GO:0060605] Subtypes: GO:1903133 References: PMID:22898778 Sources: GOC:TermGenie, GOC:dph, GO_REF:0000058 Definition: Any process that modulates the frequency, rate or extent of tube lumen cavitation.